{
  "term_id": "GO:0051864",
  "gene_name": "Ribosomal oxygenase 1",
  "term_label": "histone H3K36 demethylase activity",
  "gene": "UniProtKB:Q9H6W3",
  "gene_symbol": "RIOX1"
}